{
  "gene_name": "Receptor tyrosine-protein kinase erbB-3",
  "term_label": "positive regulation of MAPK cascade",
  "gene": "UniProtKB:P21860",
  "term_id": "GO:0043410",
  "gene_symbol": "ERBB3"
}